{
  "gene": "UniProtKB:Q9BYK8",
  "term_label": "cytosol",
  "gene_name": "Helicase with zinc finger domain 2",
  "gene_symbol": "HELZ2",
  "term_id": "GO:0005829"
}